negative regulation of calcium ion transmembrane transporter activity [GO:1901020] (biological process) Definition: Any process that stops, prevents or reduces the frequency, rate or extent of calcium ion transmembrane transporter activity. Subtypes: negative regulation of ryanodine-sensitive calcium-release channel activity [GO:0060315], negative regulation of store-operated calcium channel activity [GO:1901340], negative regulation of voltage-gated calcium channel activity [GO:1901386], negative regulation of ATPase-coupled calcium transmembrane transporter activity [GO:1901895] Also known as: down regulation of calcium ion transmembrane transporter activity, down-regulation of calcium ion transmembrane transporter activity, downregulation of calcium ion transmembrane transporter activity, inhibition of calcium ion transmembrane transporter activity Relationships: is a type of GO:0032413; is a type of negative regulation of calcium ion transmembrane transport [GO:1903170]; negatively regulates calcium ion transmembrane transporter activity [GO:0015085] Sources: GOC:BHF, GOC:TermGenie